{
  "term_id": "UNKNOWN:0003",
  "term_label": "Unknown cellular component",
  "gene": "UniProtKB:Q96L15",
  "gene_name": "Ecto-ADP-ribosyltransferase 5",
  "gene_symbol": "ART5"
}